{
  "term_label": "Unknown molecular function",
  "gene": "UniProtKB:Q53EU6",
  "term_id": "UNKNOWN:0001",
  "gene_symbol": "GPAT3",
  "gene_name": "Glycerol-3-phosphate acyltransferase 3"
}